{
  "term_id": "GO:0044344",
  "gene": "UniProtKB:Q6XUX3",
  "gene_name": "Dual serine_threonine and tyrosine protein kinase",
  "term_label": "cellular response to fibroblast growth factor stimulus",
  "gene_symbol": "DSTYK"
}